{
  "term_id": "GO:0005925",
  "gene": "UniProtKB:P05556",
  "term_label": "focal adhesion",
  "gene_name": "Integrin beta-1",
  "gene_symbol": "ITGB1"
}